{
  "term_label": "DNA replication",
  "gene_name": "Replication protein A 32 kDa subunit",
  "gene_symbol": "RPA2",
  "gene": "UniProtKB:P15927",
  "term_id": "GO:0006260"
}